mating type switching [GO:0007533] (biological process) Definition: The conversion of a single-cell organism from one mating type to another by the precise replacement of a DNA sequence at the expressed mating type locus with a copy of a sequence from a donor locus. Also known as: mating type switching and recombination Regulation: regulated by regulation of mating type switching [GO:0031494]; RO_0002212 by negative regulation of mating type switching [GO:0031495]; positively regulated by positive regulation of mating type switching [GO:0031496] References: PMID:9928492 Relationships: is a type of GO:0007531; is a type of reproductive process in single-celled organism [GO:0022413]